{
  "gene_name": "Olfactory receptor 52E4",
  "gene": "UniProtKB:Q8NGH9",
  "term_label": "plasma membrane",
  "term_id": "GO:0005886",
  "gene_symbol": "OR52E4"
}